{
  "gene_name": "Transcription factor ATOH1",
  "gene_symbol": "ATOH1",
  "term_label": "axon development",
  "gene": "UniProtKB:Q92858",
  "term_id": "GO:0061564"
}